{
  "term_id": "GO:0072092",
  "gene_name": "Kinesin-like protein KIF26B",
  "gene_symbol": "KIF26B",
  "gene": "UniProtKB:Q2KJY2",
  "term_label": "ureteric bud invasion"
}